{
  "term_id": "GO:0005576",
  "term_label": "extracellular region",
  "gene": "UniProtKB:Q8N5I4",
  "gene_name": "Dehydrogenase_reductase SDR family member on chromosome X",
  "gene_symbol": "DHRSX"
}